{
  "term_label": "cytoskeleton organization",
  "gene": "UniProtKB:Q9BY11",
  "gene_name": "Protein kinase C and casein kinase substrate in neurons protein 1",
  "term_id": "GO:0007010",
  "gene_symbol": "PACSIN1"
}